{
  "gene": "UniProtKB:P0DPA2",
  "term_label": "Unknown cellular component",
  "gene_symbol": "VSIG8",
  "term_id": "UNKNOWN:0003",
  "gene_name": "V-set and immunoglobulin domain-containing protein 8"
}